regulation of alcohol catabolic process [GO:1900419] (BP) Subtypes: GO:1900065, negative regulation of alcohol catabolic process [GO:1900420], GO:1900421 Definition: Any process that modulates the frequency, rate or extent of alcohol catabolic process within a cell. Sources: GOC:TermGenie Relationships: is a type of regulation of catabolic process [GO:0009894]; is_a regulation of small molecule metabolic process [GO:0062012]; regulates GO:0046164